{
  "gene_symbol": "RCC1",
  "term_label": "regulation of mitotic spindle assembly",
  "gene_name": "Regulator of chromosome condensation",
  "gene": "UniProtKB:P18754",
  "term_id": "GO:1901673"
}